{
  "term_id": "GO:0000978",
  "term_label": "RNA polymerase II cis-regulatory region sequence-specific DNA binding",
  "gene": "UniProtKB:Q9BQW3",
  "gene_name": "Transcription factor COE4",
  "gene_symbol": "EBF4"
}